plasma membrane-derived thylakoid membrane [GO:0031676] (cellular component) Definition: The pigmented membrane of a plasma membrane-derived thylakoid. Sources: GOC:mah, GOC:mtg_sensu Relationships: is_a GO:0042651; is a type of GO:0042717; is a type of GO:0098590; is part of bacterial thylakoid [GO:0030075] Also known as: plasma membrane thylakoid membrane